{
  "term_id": "GO:0019433",
  "gene_symbol": "LIPE",
  "gene": "UniProtKB:Q05469",
  "gene_name": "Hormone-sensitive lipase",
  "term_label": "triglyceride catabolic process"
}